L-proline catabolic process [GO:0006562] (biological process) Definition: The chemical reactions and pathways resulting in the breakdown of L-proline (pyrrolidine-2-carboxylic acid), a chiral, cyclic, nonessential alpha-amino acid found in peptide linkage in proteins. Sources: GOC:jl, ISBN:0198506732 Also known as: proline breakdown, proline catabolism, proline degradation Relationships: is a type of proline metabolic process [GO:0006560]; is a type of L-amino acid catabolic process [GO:0170035]; is_a proteinogenic amino acid catabolic process [GO:0170040] Subtypes: GO:0010133, proline catabolic process to 2-oxoglutarate [GO:0019495]